{
  "gene_name": "Zinc finger protein 559",
  "gene": "UniProtKB:Q9BR84",
  "term_id": "GO:0000981",
  "term_label": "DNA-binding transcription factor activity, RNA polymerase II-specific",
  "gene_symbol": "ZNF559"
}